{
  "gene_name": "Neutral alpha-glucosidase AB",
  "term_label": "glucosidase II complex",
  "term_id": "GO:0017177",
  "gene_symbol": "GANAB",
  "gene": "UniProtKB:Q14697"
}